SCF-Ucc1 ubiquitin ligase complex [GO:0097673] (cellular component) Relationships: is a type of SCF ubiquitin ligase complex [GO:0019005] References: PMID:14747994, PMID:25982115 Sources: GOC:jd, GOC:vw Definition: An SCF ubiquitin ligase complex in which the F-box protein is YLR224W in S. cerevisiae. Also known as: SCF-YLR224W ubiquitin ligase complex